{
  "term_id": "UNKNOWN:0001",
  "gene": "UniProtKB:A8MT33",
  "gene_symbol": "SYCE1L",
  "term_label": "Unknown molecular function",
  "gene_name": "Synaptonemal complex central element protein 1-like"
}